{
  "gene": "UniProtKB:P01225",
  "gene_name": "Follitropin subunit beta",
  "term_id": "GO:0001541",
  "gene_symbol": "FSHB",
  "term_label": "ovarian follicle development"
}